{
  "term_label": "plasma membrane",
  "gene": "UniProtKB:P21583",
  "gene_name": "Kit ligand",
  "gene_symbol": "KITLG",
  "term_id": "GO:0005886"
}